cytochrome-b5 reductase activity, acting on NADPH [GO:0090523] (molecular function) Relationships: is a type of GO:0004128 Sources: RHEA:64576 Definition: Catalysis of the reaction: 2 Fe(III)-[cytochrome b5] + NADPH = 2 Fe(II)-[cytochrome b5] + NADP+ + H+. Also known as: cytochrome-b5 reductase activity